phosphatidylinositol-4,5-bisphosphate phospholipase C activity [GO:0004435] (molecular function) Relationships: is a type of GO:0004629 Sources: RHEA:33179 Definition: Catalysis of the reaction: a 1,2-diacyl-sn-glycero-3-phospho-(1D-myo-inositol-4,5-bisphosphate) + H2O = 1D-myo-inositol 1,4,5-trisphosphate + a 1,2-diacyl-sn-glycerol + H+. Also known as: monophosphatidylinositol phosphodiesterase activity, phosphatidylinositol phospholipase C activity, triphosphoinositide phosphodiesterase activity, 1-phosphatidylinositol-4,5-bisphosphate phosphodiesterase activity, 1-phosphatidyl-1D-myo-inositol-4,5-bisphosphate inositoltrisphosphohydrolase activity, 1-phosphatidyl-D-myo-inositol-4,5-bisphosphate inositoltrisphosphohydrolase activity, PI-PLC activity, phosphatidylinositol-4,5-bisphosphate hydrolysis, phosphoinositidase C activity, phosphoinositide phospholipase C activity